{
  "gene_symbol": "PGC",
  "gene_name": "Gastricsin",
  "term_id": "GO:0004190",
  "term_label": "aspartic-type endopeptidase activity",
  "gene": "UniProtKB:P20142"
}